{
  "gene": "UniProtKB:Q9GZV7",
  "term_id": "GO:0005615",
  "term_label": "extracellular space",
  "gene_name": "Hyaluronan and proteoglycan link protein 2",
  "gene_symbol": "HAPLN2"
}